{
  "gene_name": "Interferon-related developmental regulator 1",
  "term_id": "UNKNOWN:0001",
  "gene_symbol": "IFRD1",
  "term_label": "Unknown molecular function",
  "gene": "UniProtKB:O00458"
}